aromatic primary alcohol biosynthetic process [GO:1902655] (biological process) Definition: The chemical reactions and pathways resulting in the formation of aromatic primary alcohol. References: PMID:19219878 Sources: GOC:TermGenie, GOC:mengo_curators, GO_REF:0000068 Relationships: is a type of GO:0034309; is a type of aromatic primary alcohol metabolic process [GO:1902654] Also known as: aromatic primary alcohol anabolism, aromatic primary alcohol biosynthesis, aromatic primary alcohol formation, aromatic primary alcohol synthesis